{
  "gene": "UniProtKB:Q5VYY2",
  "gene_name": "Lipase member M",
  "term_label": "lipase activity",
  "term_id": "GO:0016298",
  "gene_symbol": "LIPM"
}